multi-pass transmembrane protein insertion into ER membrane [GO:0160063] (biological process) Relationships: is a type of GO:0045048 References: PMID:36261522, PMID:36261528 Definition: A process of protein insertion of multi-pass membrane proteins into the endoplasmic reticulum (ER) membrane. Insertion of multi-pass membrane proteins is mediated by the multi-pass translocon complex and takes place following membrane insertion of the first few transmembrane segments of proteins by the SEC61 complex to promote insertion of subsequent transmembrane regions.